(S)-limonene 7-monooxygenase activity [GO:0018676] (molecular function) Relationships: is a type of GO:0016712; is a type of limonene monooxygenase activity [GO:0019113] Also known as: (-)-limonene 7-monooxygenase activity Sources: RHEA:23432 Definition: Catalysis of the reaction: (4S)-limonene + O2 + reduced [NADPH--hemoprotein reductase] = (4S)-perillyl alcohol + H+ + H2O + oxidized [NADPH--hemoprotein reductase].